tRNA (guanosine(9)-N1)-methyltransferase activity [GO:0052905] (molecular function) Also known as: tRNA (guanine(9)-N(1))-methyltransferase activity, tRNA (guanosine(9)-N(1))-methyltransferase activity, tRNA (guanosine(9)-N1-)-methyltransferase activity, tRNA (guanine-N(1)-)-methyltransferase activity, tRNA m(1)G(9) Mtase activity, tRNA m(1)G(9)-methyltransferase activity, tRNA(m(1)G(9)/m(1)A(9))-methyltransferase activity, tRNA(m(1)G(9)/m(1)A(9))Mtase activity Definition: Catalysis of the reaction: guanosine9 in tRNA + S-adenosyl-L-methionine = H+ + N1-methylguanosine9 in tRNA + S-adenosyl-L-homocysteine. Relationships: is a type of tRNA (guanine) methyltransferase activity [GO:0016423] Sources: RHEA:43156